{
  "term_id": "GO:0034236",
  "term_label": "protein kinase A catalytic subunit binding",
  "gene": "UniProtKB:P10644",
  "gene_symbol": "PRKAR1A",
  "gene_name": "cAMP-dependent protein kinase type I-alpha regulatory subunit"
}